{
  "gene_name": "Methionine adenosyltransferase 2 subunit beta",
  "term_label": "S-adenosylmethionine biosynthetic process",
  "gene_symbol": "MAT2B",
  "term_id": "GO:0006556",
  "gene": "UniProtKB:Q9NZL9"
}